D-glucose uniporter activity [GO:0015304] (molecular function) Definition: Enables the transfer of a solute or solutes from one side of a membrane to the other according to the reaction: D-glucose(out) = D-glucose(in). Sources: TC:2.A.1.1.12, TC:2.A.1.1.4, TC:2.A.1.1.6 Also known as: glucose uniporter activity, galactose, glucose uniporter activity Relationships: is a type of hexose uniporter activity [GO:0008516]; is_a D-glucose transmembrane transporter activity [GO:0055056]